{
  "term_label": "cell-matrix adhesion",
  "gene_name": "Mesothelin-like protein",
  "gene": "UniProtKB:Q96KJ4",
  "term_id": "GO:0007160",
  "gene_symbol": "MSLNL"
}